DN3 thymocyte differentiation [GO:1904156] (biological process) Relationships: is a type of GO:0033077 Definition: The process in which a relatively unspecialized cell acquires the specialized features of a DN3 thymocyte. A DN3 thymocyte is a CD4-,CD8- thymocyte that is also CD44+,CD25+. References: PMID:25398325 Sources: GOC:TermGenie, GOC:dph, GO_REF:0000086